regulation of establishment of protein localization to mitochondrion [GO:1903747] (BP) Definition: Any process that modulates the frequency, rate or extent of establishment of protein localization to mitochondrion. Subtypes: regulation of protein targeting to mitochondrion [GO:1903214], negative regulation of establishment of protein localization to mitochondrion [GO:1903748], positive regulation of establishment of protein localization to mitochondrion [GO:1903749] References: PMID:16857185 Sources: GOC:TermGenie, GO_REF:0000058 Also known as: regulation of establishment of protein localisation to mitochondrion, regulation of establishment of protein localization in mitochondrion Relationships: is a type of regulation of establishment of protein localization [GO:0070201]; regulates GO:0072655